positive regulation of T cell proliferation [GO:0042102] (biological process) Definition: Any process that activates or increases the rate or extent of T cell proliferation. Sources: GOC:ai Also known as: positive regulation of T lymphocyte proliferation, positive regulation of T-lymphocyte proliferation, up regulation of T cell proliferation, up-regulation of T cell proliferation, upregulation of T cell proliferation, activation of T cell proliferation, stimulation of T cell proliferation Relationships: is a type of GO:0042129; is a type of positive regulation of lymphocyte proliferation [GO:0050671]; is a type of GO:0050870; RO_0002213 GO:0042098 Subtypes: GO:0033091, GO:0042103, GO:0042104, positive regulation of alpha-beta T cell proliferation [GO:0046641], GO:0046648